calmodulin binding [GO:0005516] (molecular function) Sources: GOC:krc Relationships: is a type of protein binding [GO:0005515] Definition: Binding to calmodulin, a calcium-binding protein with many roles, both in the calcium-bound and calcium-free states.